{
  "gene_symbol": "STX5",
  "term_id": "GO:0000139",
  "term_label": "Golgi membrane",
  "gene": "UniProtKB:Q13190",
  "gene_name": "Syntaxin-5"
}